{
  "gene_name": "Ankyrin repeat and BTB_POZ domain-containing protein 1",
  "gene": "UniProtKB:Q969K4",
  "gene_symbol": "ABTB1",
  "term_label": "Unknown biological process",
  "term_id": "UNKNOWN:0002"
}